{
  "gene_symbol": "CEP68",
  "term_id": "UNKNOWN:0003",
  "term_label": "Unknown cellular component",
  "gene": "UniProtKB:Q76N32",
  "gene_name": "Centrosomal protein of 68 kDa"
}